{
  "gene_symbol": "OR7G1",
  "gene": "UniProtKB:Q8NGA0",
  "gene_name": "Olfactory receptor 7G1",
  "term_label": "plasma membrane",
  "term_id": "GO:0005886"
}